{
  "term_label": "Unknown biological process",
  "term_id": "UNKNOWN:0002",
  "gene_symbol": "PRR20A",
  "gene": "UniProtKB:P86496",
  "gene_name": "Proline-rich protein 20A"
}